{
  "gene": "UniProtKB:Q9UJK0",
  "term_id": "UNKNOWN:0003",
  "term_label": "Unknown cellular component",
  "gene_symbol": "TSR3",
  "gene_name": "18S rRNA aminocarboxypropyltransferase"
}